{
  "gene": "UniProtKB:Q00987",
  "term_label": "cytoplasm",
  "gene_symbol": "MDM2",
  "gene_name": "E3 ubiquitin-protein ligase Mdm2",
  "term_id": "GO:0005737"
}